{
  "gene_symbol": "PGGT1B",
  "term_id": "GO:0005953",
  "term_label": "CAAX-protein geranylgeranyltransferase complex",
  "gene": "UniProtKB:P53609",
  "gene_name": "Geranylgeranyl transferase type-1 subunit beta"
}